{
  "gene": "UniProtKB:Q8NGE2",
  "gene_name": "Olfactory receptor 2AP1",
  "term_label": "Unknown biological process",
  "term_id": "UNKNOWN:0002",
  "gene_symbol": "OR2AP1"
}